{
  "term_id": "GO:0034314",
  "gene_name": "Actin-related protein 2_3 complex subunit 2",
  "gene": "UniProtKB:O15144",
  "term_label": "Arp2/3 complex-mediated actin nucleation",
  "gene_symbol": "ARPC2"
}